positive regulation of insulin receptor signaling pathway by insulin receptor internalization [GO:0038015] (biological process) Also known as: positive regulation of insulin receptor signalling pathway by insulin receptor internalization Definition: Any process in which internalization of an insulin receptor activates or increases the frequency, rate or extent of the insulin receptor signaling pathway. Endocytosis of activated receptors can concentrate receptors within endosomes and allow the insulin receptor to phosphorylate substrates that are spatially distinct from those accessible at the plasma membrane. References: PMID:9609114 Sources: GOC:bf, GOC:signaling Relationships: is a type of GO:0038010; is a type of insulin receptor internalization [GO:0038016]; is_a positive regulation of insulin receptor signaling pathway [GO:0046628]